{
  "gene": "UniProtKB:P13688",
  "gene_symbol": "CEACAM1",
  "term_label": "plasma membrane",
  "gene_name": "Carcinoembryonic antigen-related cell adhesion molecule 1",
  "term_id": "GO:0005886"
}